{
  "term_label": "RNA polymerase II cis-regulatory region sequence-specific DNA binding",
  "gene_symbol": "SKOR1",
  "gene": "UniProtKB:P84550",
  "term_id": "GO:0000978",
  "gene_name": "SKI family transcriptional corepressor 1"
}